DNA synthesis involved in mitochondrial DNA replication [GO:0110166] (biological process) Also known as: DNA biosynthetic process involved in mitochondrial DNA replication Relationships: is a type of GO:0032042; is a type of GO:0090592; is part of mitochondrial DNA replication [GO:0006264] References: PMID:28408491, PMID:29931097 Definition: Any DNA biosynthetic process that is involved in mitochondrial DNA replication.